{
  "gene_symbol": "FOXO6",
  "gene_name": "Forkhead box protein O6",
  "term_id": "GO:0005634",
  "term_label": "nucleus",
  "gene": "UniProtKB:A8MYZ6"
}